{
  "term_label": "mitotic G1/S transition checkpoint signaling",
  "gene": "UniProtKB:Q9H4B4",
  "gene_symbol": "PLK3",
  "gene_name": "Serine_threonine-protein kinase PLK3",
  "term_id": "GO:0044819"
}